deacetylipecoside synthase activity [GO:0050557] (molecular function) Relationships: is a type of hydrolase activity, acting on carbon-nitrogen (but not peptide) bonds [GO:0016810] Definition: Catalysis of the reaction: deacetylipecoside + H2O = dopamine + secologanin. Sources: RHEA:12296 Also known as: deacetylipecoside dopamine-lyase (secologanin-forming), deacetylipecoside dopamine-lyase activity